postsynaptic specialization, intracellular component [GO:0099091] (cellular component) Sources: GOC:dos Subtypes: postsynaptic density, intracellular component [GO:0099092], postsynaptic specialization of symmetric synapse, intracellular component [GO:0099165] Definition: A network of proteins adjacent to the postsynaptic membrane. Its major components include the proteins that spatially and functionally organize neurotransmitter receptors in the adjacent membrane, such as anchoring and scaffolding molecules, signaling enzymes and cytoskeletal components. Relationships: is a type of intracellular membraneless organelle [GO:0043232]; is part of postsynaptic specialization [GO:0099572]